{
  "gene_symbol": "CARNS1",
  "gene_name": "Carnosine synthase 1",
  "gene": "UniProtKB:A5YM72",
  "term_label": "Unknown cellular component",
  "term_id": "UNKNOWN:0003"
}